potassium ion transport [GO:0006813] (BP) Relationships: is a type of metal ion transport [GO:0030001] Definition: The directed movement of potassium ions (K+) into, out of or within a cell, or between cells, by means of some agent such as a transporter or pore. Subtypes: potassium ion transmembrane transport [GO:0071805] Sources: GOC:ai Regulation: regulated by regulation of potassium ion transport [GO:0043266]; negatively regulated by negative regulation of potassium ion transport [GO:0043267]; positively regulated by GO:0043268 Also known as: sodium/potassium transport, cellular potassium ion transport, potassium conductance, potassium ion conductance, K+ conductance, low voltage-dependent potassium channel auxiliary protein activity, low voltage-gated potassium channel auxiliary protein activity, potassium transport